protein methylesterase activity [GO:0051723] (molecular function) Subtypes: protein-glutamate methylesterase activity [GO:0008984], prenylcysteine methylesterase activity [GO:0010296] Definition: Catalysis of the reaction: protein amino acid methyl ester + H2O = protein amino acid + methanol. Also known as: protein carboxylic ester hydrolase activity, PME activity, protein carboxyl methylesterase activity, protein methyl-esterase activity Relationships: is a type of GO:0052689; is a type of catalytic activity, acting on a protein [GO:0140096] Sources: GOC:ai